polysaccharide O-methyltransferase activity [GO:0030734] (molecular function) Also known as: S-adenosyl-L-methionine:1,4-alpha-D-glucan 6-O-methyltransferase activity, acylpolysacharide 6-methyltransferase activity, polysaccharide methyltransferase activity Definition: Catalysis of the reaction: S-adenosyl-L-methionine + 1,4-N1-D-glucooligosaccharide = S-adenosyl-L-homocysteine + oligosaccharide containing 6-methyl-D-glucose units. Sources: EC:2.1.1.18 Relationships: is a type of S-adenosylmethionine-dependent methyltransferase activity [GO:0008757]